{
  "term_label": "poly(A) binding",
  "gene": "UniProtKB:Q13310",
  "term_id": "GO:0008143",
  "gene_name": "Polyadenylate-binding protein 4",
  "gene_symbol": "PABPC4"
}